positive regulation of skeletal muscle fiber development [GO:0048743] (BP) Definition: Any process that activates, maintains or increases the rate of skeletal muscle fiber development. Muscle fibers are formed by the maturation of myotubes. They can be classed as slow, intermediate/fast or fast. Also known as: positive regulation of skeletal muscle fibre development, positive regulation of skeletal myofiber development, positive regulation of skeletal myofibre development, up regulation of skeletal muscle fiber development, up-regulation of skeletal muscle fiber development, upregulation of skeletal muscle fiber development, activation of skeletal muscle fiber development, stimulation of skeletal muscle fiber development Relationships: is a type of positive regulation of cell development [GO:0010720]; is a type of positive regulation of skeletal muscle tissue development [GO:0048643]; is a type of regulation of skeletal muscle fiber development [GO:0048742]; is a type of positive regulation of striated muscle cell differentiation [GO:0051155]; positively regulates skeletal muscle fiber development [GO:0048741] Sources: GOC:dph, GOC:jid, GOC:lm, GOC:mtg_muscle